male meiotic nuclear division [GO:0007140] (biological process) Also known as: male nuclear division, male meiosis Definition: A cell cycle process by which the cell nucleus divides as part of a meiotic cell cycle in the male germline. Relationships: is_a GO:0140013; is part of male gamete generation [GO:0048232] Sources: GOC:dph, GOC:mah, GOC:vw Subtypes: GO:0007141, male meiosis II [GO:0007142]